response to rhamnose [GO:0032149] (biological process) Relationships: is a type of response to hexose [GO:0009746] Subtypes: cellular response to rhamnose stimulus [GO:0071334] Definition: Any process that results in a change in state or activity of a cell or an organism (in terms of movement, secretion, enzyme production, gene expression, etc.) as a result of a rhamnose stimulus. Also known as: response to rhamnose stimulus, response to L-rhamnose stimulus Sources: GOC:mlg